{
  "gene": "UniProtKB:Q9NSC5",
  "gene_symbol": "HOMER3",
  "term_id": "GO:0014069",
  "term_label": "postsynaptic density",
  "gene_name": "Homer protein homolog 3"
}